{
  "gene": "UniProtKB:Q8NGX3",
  "term_id": "GO:0004984",
  "gene_name": "Olfactory receptor 10T2",
  "term_label": "olfactory receptor activity",
  "gene_symbol": "OR10T2"
}